{
  "gene_symbol": "CALML5",
  "gene_name": "Calmodulin-like protein 5",
  "term_label": "microtubule cytoskeleton organization",
  "gene": "UniProtKB:Q9NZT1",
  "term_id": "GO:0000226"
}